{
  "gene_name": "Putative synaptogyrin-2 like protein",
  "term_label": "neuromuscular junction",
  "gene_symbol": "A8MWL6",
  "term_id": "GO:0031594",
  "gene": "UniProtKB:A8MWL6"
}